{
  "gene_symbol": "CHRNA5",
  "gene": "UniProtKB:P30532",
  "gene_name": "Neuronal acetylcholine receptor subunit alpha-5",
  "term_label": "monoatomic ion transmembrane transport",
  "term_id": "GO:0034220"
}